{
  "term_id": "GO:0004984",
  "gene_name": "Olfactory receptor 5AS1",
  "term_label": "olfactory receptor activity",
  "gene": "UniProtKB:Q8N127",
  "gene_symbol": "OR5AS1"
}